{
  "gene": "UniProtKB:P52435",
  "gene_name": "DNA-directed RNA polymerase II subunit RPB11-a",
  "term_id": "GO:0003899",
  "term_label": "DNA-directed RNA polymerase activity",
  "gene_symbol": "POLR2J"
}